{
  "term_label": "actin filament depolymerization",
  "term_id": "GO:0030042",
  "gene_name": "Twinfilin-1",
  "gene_symbol": "TWF1",
  "gene": "UniProtKB:Q12792"
}